{
  "gene": "UniProtKB:Q13156",
  "gene_name": "Replication protein A 30 kDa subunit",
  "term_id": "GO:0006289",
  "term_label": "nucleotide-excision repair",
  "gene_symbol": "RPA4"
}